{
  "term_label": "positive regulation of autophagy",
  "gene": "UniProtKB:Q5S007",
  "term_id": "GO:0010508",
  "gene_name": "Leucine-rich repeat serine_threonine-protein kinase 2",
  "gene_symbol": "LRRK2"
}